rhombomere 8 development [GO:0021574] (biological process) Relationships: is a type of rhombomere development [GO:0021546] Definition: The process whose specific outcome is the progression of rhombomere 8 over time, from its formation to the mature structure. Rhombomeres are transverse segments of the developing rhombencephalon. Rhombomeres are lineage restricted, express different genes from one another, and adopt different developmental fates. Rhombomeres are numbered in anterior to posterior order. Sources: GOC:cls, GOC:curators, GOC:dgh, GOC:dph, GOC:jid